{
  "term_id": "UNKNOWN:0001",
  "term_label": "Unknown molecular function",
  "gene": "UniProtKB:Q7Z5D8",
  "gene_name": "NANOG neighbor homeobox",
  "gene_symbol": "NANOGNB"
}